{
  "term_id": "UNKNOWN:0002",
  "gene_name": "Glioma pathogenesis-related protein 1",
  "term_label": "Unknown biological process",
  "gene": "UniProtKB:P48060",
  "gene_symbol": "GLIPR1"
}